{
  "gene_symbol": "ITPR1",
  "gene": "UniProtKB:Q14643",
  "gene_name": "Inositol 1,4,5-trisphosphate receptor type 1",
  "term_id": "GO:0016529",
  "term_label": "sarcoplasmic reticulum"
}